cheating during chimeric sorocarp development [GO:0099139] (biological process) Definition: Any process during chimeric sorocarp development that increases by which a cell increases the number of spore cells sharing its genotype at the expense of cells of other genotypes. Relationships: is a type of regulation of sorocarp spore cell differentiation [GO:1901261]; is part of chimeric sorocarp development [GO:0099134] References: PMID:18272966